{
  "gene": "UniProtKB:Q7Z5Q1",
  "term_label": "synapse",
  "gene_name": "Cytoplasmic polyadenylation element-binding protein 2",
  "gene_symbol": "CPEB2",
  "term_id": "GO:0045202"
}